{
  "gene_symbol": "DCBLD1",
  "term_id": "GO:0038023",
  "gene_name": "Discoidin, CUB and LCCL domain-containing protein 1",
  "gene": "UniProtKB:Q8N8Z6",
  "term_label": "signaling receptor activity"
}